{
  "gene_symbol": "GPR32P1",
  "term_id": "GO:0002430",
  "gene": "UniProtKB:Q8NGA4",
  "gene_name": "Putative G-protein coupled receptor GPR32P1",
  "term_label": "complement receptor mediated signaling pathway"
}